{
  "term_label": "Wnt-protein binding",
  "gene": "UniProtKB:Q9H461",
  "gene_symbol": "FZD8",
  "term_id": "GO:0017147",
  "gene_name": "Frizzled-8"
}